exit from dormancy [GO:0097438] (biological process) Also known as: release from dormancy Subtypes: release of seed from dormancy [GO:0048838] Sources: GOC:PO_curators, PO_REF:00009 Definition: The dormancy process that results in exit from dormancy. Dormancy (sometimes called a dormant state) is a suspension of most physiological activity and growth that can be reactivated. Relationships: is a type of dormancy process [GO:0022611]